exosomal secretion [GO:1990182] (biological process) Definition: The process whereby a membrane-bounded vesicle is released into the extracellular region by fusion of the limiting endosomal membrane of a multivesicular body with the plasma membrane. References: PMID:10572093, PMID:12154376, PMID:16773132, PMID:18617898 Sources: GOC:hjd Regulation: regulated by GO:1903541; negatively regulated by GO:1903542; positively regulated by GO:1903543 Also known as: exosomal secretory pathway, extracellular vesicular exosome secretion, multi-vesicular body fusion with plasma membrane, secretion of exosome, exosomal protein secretion Relationships: is a type of exocytosis [GO:0006887]; is_a establishment of vesicle localization [GO:0051650]; BFO_0000050 extracellular exosome biogenesis [GO:0097734]